{
  "gene": "UniProtKB:Q9NWF9",
  "term_label": "Unknown biological process",
  "term_id": "UNKNOWN:0002",
  "gene_symbol": "RNF216",
  "gene_name": "E3 ubiquitin-protein ligase RNF216"
}